{
  "term_label": "poly(A) binding",
  "gene": "UniProtKB:Q6PJT7",
  "gene_name": "Zinc finger CCCH domain-containing protein 14",
  "term_id": "GO:0008143",
  "gene_symbol": "ZC3H14"
}